{
  "gene_symbol": "MS4A3",
  "term_label": "Unknown biological process",
  "term_id": "UNKNOWN:0002",
  "gene": "UniProtKB:Q96HJ5",
  "gene_name": "Membrane-spanning 4-domains subfamily A member 3"
}